diadenosine polyphosphate catabolic process [GO:0015961] (biological process) Definition: The chemical reactions and pathways resulting in the breakdown of diadenosine polyphosphate, a derivative of the nucleoside adenosine with phosphate groups attached. Sources: GOC:ai Also known as: diadenosine polyphosphate breakdown, diadenosine polyphosphate catabolism, diadenosine polyphosphate degradation Relationships: is a type of nucleotide catabolic process [GO:0009166]; is a type of diadenosine polyphosphate metabolic process [GO:0015959] Subtypes: diadenosine triphosphate catabolic process [GO:0015964], diadenosine tetraphosphate catabolic process [GO:0015967], GO:1901907, diadenosine hexaphosphate catabolic process [GO:1901909]